regulation of intermediate mesodermal cell fate specification [GO:0048399] (biological process) Definition: Any process that modulates the frequency, rate or extent of intermediate mesoderm cell fate specification. Sources: GOC:dgh Relationships: is a type of GO:0042661; regulates intermediate mesodermal cell fate specification [GO:0048398] Subtypes: positive regulation of intermediate mesodermal cell fate specification [GO:0048400], GO:0048401